5-methyltetrahydropteroyltri-L-glutamate-dependent methyltransferase activity [GO:0042085] (molecular function) Definition: Catalysis of the transfer of a methyl group to an acceptor molecule; dependent on the presence of 5-methyltetrahydropteroyltri-L-glutamate. Sources: GOC:ai Relationships: is a type of methyltransferase activity [GO:0008168] Subtypes: 5-methyltetrahydropteroyltriglutamate-homocysteine S-methyltransferase activity [GO:0003871]